re-entry into mitotic cell cycle after pheromone arrest [GO:0000321] (biological process) Definition: The resumption of the mitotic cell division cycle by pheromone-arrested cells that have not mated. An example of this process is found in Saccharomyces cerevisiae. Relationships: is a type of re-entry into mitotic cell cycle [GO:0000320]; is a type of GO:0000754 References: PMID:9927449 Sources: GOC:krc